{
  "gene_name": "Polypeptide N-acetylgalactosaminyltransferase 10",
  "gene": "UniProtKB:Q86SR1",
  "term_id": "GO:0004653",
  "term_label": "polypeptide N-acetylgalactosaminyltransferase activity",
  "gene_symbol": "GALNT10"
}